{
  "gene_symbol": "ERH",
  "term_label": "Unknown molecular function",
  "gene_name": "Enhancer of rudimentary homolog",
  "term_id": "UNKNOWN:0001",
  "gene": "UniProtKB:P84090"
}